{
  "gene": "UniProtKB:Q96L46",
  "term_label": "calpain complex",
  "term_id": "GO:0110158",
  "gene_symbol": "CAPNS2",
  "gene_name": "Calpain small subunit 2"
}